{
  "term_id": "GO:0051897",
  "term_label": "positive regulation of phosphatidylinositol 3-kinase/protein kinase B signal transduction",
  "gene": "UniProtKB:Q9GZP0",
  "gene_name": "Platelet-derived growth factor D",
  "gene_symbol": "PDGFD"
}